{
  "gene": "UniProtKB:P14672",
  "gene_name": "Solute carrier family 2, facilitated glucose transporter member 4",
  "term_id": "GO:0046323",
  "term_label": "D-glucose import",
  "gene_symbol": "SLC2A4"
}